{
  "term_label": "N-acylneuraminate-9-phosphatase activity",
  "gene": "UniProtKB:Q8TBE9",
  "term_id": "GO:0050124",
  "gene_symbol": "NANP",
  "gene_name": "N-acylneuraminate-9-phosphatase"
}